aerobic phenol-containing compound biosynthetic process [GO:0046190] (biological process) Definition: The chemical reactions and pathways resulting in the formation of a phenol, any compound containing one or more hydroxyl groups directly attached to an aromatic carbon ring, in the presence of oxygen. Relationships: is a type of phenol-containing compound biosynthetic process [GO:0046189] Sources: GOC:ai Also known as: aerobic phenol-containing compound anabolism, aerobic phenol-containing compound biosynthesis, aerobic phenol-containing compound formation, aerobic phenol-containing compound synthesis